stomatal opening [GO:1990069] (biological process) Definition: The process of opening of stomata, pores in the epidermis of leaves and stems bordered by two guard cells and serving in gas exchange. References: PMID:21749899 Relationships: is a type of stomatal movement [GO:0010118] Regulation: regulated by regulation of stomatal opening [GO:1902456]; negatively regulated by negative regulation of stomatal opening [GO:1902457]; RO_0002213 by positive regulation of stomatal opening [GO:1902458]